{
  "gene_name": "CD109 antigen",
  "gene": "UniProtKB:Q6YHK3",
  "gene_symbol": "CD109",
  "term_label": "Unknown biological process",
  "term_id": "UNKNOWN:0002"
}